{
  "gene": "UniProtKB:P12018",
  "gene_name": "Immunoglobulin iota chain",
  "term_id": "GO:0006955",
  "gene_symbol": "VPREB1",
  "term_label": "immune response"
}